{
  "gene": "UniProtKB:Q9NZS9",
  "gene_symbol": "BFAR",
  "term_id": "UNKNOWN:0003",
  "gene_name": "Bifunctional apoptosis regulator",
  "term_label": "Unknown cellular component"
}